{
  "gene_name": "Paired amphipathic helix protein Sin3b",
  "term_id": "GO:0070822",
  "gene_symbol": "SIN3B",
  "term_label": "Sin3-type complex",
  "gene": "UniProtKB:O75182"
}